{
  "gene": "UniProtKB:Q9Y5Y9",
  "term_id": "GO:0086002",
  "gene_symbol": "SCN10A",
  "term_label": "cardiac muscle cell action potential involved in contraction",
  "gene_name": "Sodium channel protein type 10 subunit alpha"
}